{
  "gene_name": "Transcription factor SOX-8",
  "gene": "UniProtKB:P57073",
  "term_label": "nucleus",
  "gene_symbol": "SOX8",
  "term_id": "GO:0005634"
}